{
  "gene_name": "KN motif and ankyrin repeat domain-containing protein 3",
  "gene": "UniProtKB:Q6NY19",
  "term_label": "Unknown molecular function",
  "term_id": "UNKNOWN:0001",
  "gene_symbol": "KANK3"
}